{
  "term_label": "extracellular space",
  "gene": "UniProtKB:P09681",
  "gene_symbol": "GIP",
  "gene_name": "Gastric inhibitory polypeptide",
  "term_id": "GO:0005615"
}